antigen processing and presentation of peptide or polysaccharide antigen via MHC class II [GO:0002504] (biological process) Relationships: is a type of antigen processing and presentation [GO:0019882] References: PMID:15531770, PMID:15771591, PMID:16153240 Sources: GOC:add, ISBN:0781735149 Also known as: peptide or polysaccharide antigen processing and presentation of via MHC class II Subtypes: GO:0002495, antigen processing and presentation of polysaccharide antigen via MHC class II [GO:0002505] Regulation: regulated by regulation of antigen processing and presentation of peptide or polysaccharide antigen via MHC class II [GO:0002580]; negatively regulated by GO:0002581; positively regulated by positive regulation of antigen processing and presentation of peptide or polysaccharide antigen via MHC class II [GO:0002582] Definition: The process in which an antigen-presenting cell expresses antigen (peptide or polysaccharide) on its cell surface in association with an MHC class II protein complex.